{
  "term_id": "GO:0005634",
  "term_label": "nucleus",
  "gene": "UniProtKB:A1L3X4",
  "gene_name": "Putative metallothionein MT1DP",
  "gene_symbol": "MT1DP"
}